protein arginylation [GO:0016598] (BP) References: PMID:17896865 Also known as: protein amino acid arginylation Relationships: is a type of protein modification process [GO:0036211]; BFO_0000050 ubiquitin-dependent protein catabolic process [GO:0006511] Definition: The conjugation of arginine to the N-terminal aspartate or glutamate of a protein; required for the degradation of the protein via the ubiquitin pathway.